amino sugar catabolic process [GO:0046348] (biological process) Subtypes: GO:0019262, GO:0030392, mannosamine catabolic process [GO:0046346], GO:1901072 Sources: GOC:curators Relationships: is a type of amino sugar metabolic process [GO:0006040]; is a type of carbohydrate derivative catabolic process [GO:1901136] Definition: The chemical reactions and pathways resulting in the breakdown of any amino sugar, sugars containing an amino group in place of a hydroxyl group. Also known as: amino sugar breakdown, amino sugar catabolism, amino sugar degradation, aminosaccharide catabolic process, aminosaccharide catabolism